{
  "gene_symbol": "XKR9",
  "gene": "UniProtKB:Q5GH70",
  "term_label": "Unknown biological process",
  "gene_name": "XK-related protein 9",
  "term_id": "UNKNOWN:0002"
}